{
  "term_label": "Unknown cellular component",
  "gene_name": "Zinc finger TRAF-type-containing protein 1",
  "gene_symbol": "ZFTRAF1",
  "gene": "UniProtKB:P0DTL6",
  "term_id": "UNKNOWN:0003"
}